{
  "term_id": "GO:0001503",
  "gene": "UniProtKB:Q9BQB4",
  "gene_name": "Sclerostin",
  "gene_symbol": "SOST",
  "term_label": "ossification"
}